cytoplasmic actin-based contraction involved in rearward cell motility [GO:0060329] (biological process) Also known as: cytoplasmic actin-based contraction involved in rearward cell locomotion Sources: GOC:dph Relationships: is a type of cytoplasmic actin-based contraction involved in cell motility [GO:0060327] Definition: The actin filament-based movement by which cytoplasmic actin filaments slide past one another resulting in a contraction that propels the cell in the direction that has been defined as the rear of the cell.